{
  "gene_name": "T-cell acute lymphocytic leukemia protein 2",
  "term_id": "GO:0006357",
  "gene_symbol": "TAL2",
  "term_label": "regulation of transcription by RNA polymerase II",
  "gene": "UniProtKB:Q16559"
}